{
  "term_label": "Unknown cellular component",
  "gene_name": "Phosphopentomutase",
  "gene_symbol": "PGM2",
  "term_id": "UNKNOWN:0003",
  "gene": "UniProtKB:Q96G03"
}